{
  "gene": "UniProtKB:Q02413",
  "gene_name": "Desmoglein-1",
  "gene_symbol": "DSG1",
  "term_id": "GO:0098609",
  "term_label": "cell-cell adhesion"
}